{
  "gene": "UniProtKB:O75901",
  "gene_name": "Ras association domain-containing protein 9",
  "gene_symbol": "RASSF9",
  "term_label": "trans-Golgi network transport vesicle membrane",
  "term_id": "GO:0012510"
}